positive regulation of reverse cholesterol transport [GO:1903064] (biological process) Also known as: up regulation of reverse cholesterol transport, up-regulation of reverse cholesterol transport, upregulation of reverse cholesterol transport, activation of reverse cholesterol transport Relationships: is a type of positive regulation of cholesterol transport [GO:0032376]; is a type of GO:1903062; positively regulates reverse cholesterol transport [GO:0043691] References: PMID:23931754 Sources: GOC:BHF, GOC:TermGenie, GOC:rl, GO_REF:0000058 Definition: Any process that activates or increases the frequency, rate or extent of reverse cholesterol transport.